positive regulation of macrophage proliferation [GO:0120041] (biological process) Relationships: is_a positive regulation of leukocyte proliferation [GO:0070665]; is a type of regulation of macrophage proliferation [GO:0120040]; positively regulates GO:0061517 Sources: GOC:BHF, GOC:BHF_miRNA, GOC:rph Definition: Any process that activates or increases the frequency, rate or extent of macrophage proliferation.